{
  "gene_name": "Ubiquitin carboxyl-terminal hydrolase 34",
  "gene": "UniProtKB:Q70CQ2",
  "term_label": "regulation of protein stability",
  "term_id": "GO:0031647",
  "gene_symbol": "USP34"
}